{
  "gene_name": "Testis-specific Y-encoded-like protein 1",
  "gene_symbol": "TSPYL1",
  "gene": "UniProtKB:Q9H0U9",
  "term_label": "chromatin",
  "term_id": "GO:0000785"
}